{
  "term_id": "GO:0006006",
  "gene_symbol": "FBN2",
  "term_label": "glucose metabolic process",
  "gene_name": "Fibrillin-2",
  "gene": "UniProtKB:P35556"
}